muconate cycloisomerase activity [GO:0018849] (molecular function) Definition: Catalysis of the reaction: 2,5-dihydro-5-oxofuran-2-acetate = cis,cis-hexadienedioate. Sources: RHEA:30031 Relationships: is a type of GO:0016872 Also known as: cis,cis-muconate cycloisomerase activity, cis,cis-muconate-lactonizing enzyme, muconate cycloisomerase I activity, muconate lactonizing enzyme I activity, muconate lactonizing enzyme activity